{
  "gene": "UniProtKB:Q9UKT9",
  "term_label": "DNA-binding transcription factor activity",
  "gene_symbol": "IKZF3",
  "term_id": "GO:0003700",
  "gene_name": "Zinc finger protein Aiolos"
}